{
  "gene_symbol": "EPS8L1",
  "gene_name": "Epidermal growth factor receptor kinase substrate 8-like protein 1",
  "gene": "UniProtKB:Q8TE68",
  "term_id": "GO:0005886",
  "term_label": "plasma membrane"
}